{
  "gene_symbol": "GRIA2",
  "gene": "UniProtKB:P42262",
  "gene_name": "Glutamate receptor 2",
  "term_id": "GO:0050804",
  "term_label": "modulation of chemical synaptic transmission"
}